{
  "term_label": "Unknown molecular function",
  "gene_symbol": "CCDC188",
  "term_id": "UNKNOWN:0001",
  "gene_name": "Coiled-coil domain-containing protein 188",
  "gene": "UniProtKB:H7C350"
}